{
  "gene": "UniProtKB:Q9H7L2",
  "term_label": "immune response-inhibiting cell surface receptor signaling pathway",
  "gene_name": "Putative killer cell immunoglobulin-like receptor-like protein KIR3DX1",
  "term_id": "GO:0002767",
  "gene_symbol": "KIR3DX1"
}